{
  "gene_name": "Transcription factor BTF3 homolog 4",
  "term_label": "Unknown cellular component",
  "gene": "UniProtKB:Q96K17",
  "term_id": "UNKNOWN:0003",
  "gene_symbol": "BTF3L4"
}